{
  "gene_name": "Angiomotin-like protein 1",
  "gene_symbol": "AMOTL1",
  "term_id": "GO:0003365",
  "gene": "UniProtKB:Q8IY63",
  "term_label": "establishment of cell polarity involved in ameboidal cell migration"
}